{
  "gene_symbol": "SVIP",
  "gene": "UniProtKB:Q8NHG7",
  "term_label": "Unknown molecular function",
  "term_id": "UNKNOWN:0001",
  "gene_name": "Small VCP_p97-interacting protein"
}